{
  "gene_name": "UPF0711 protein C18orf21",
  "term_id": "UNKNOWN:0003",
  "gene": "UniProtKB:Q32NC0",
  "term_label": "Unknown cellular component",
  "gene_symbol": "C18orf21"
}